host cell endoplasmic reticulum-Golgi intermediate compartment [GO:0044172] (cellular component) Definition: A complex system of membrane-bounded compartments located between host cell endoplasmic reticulum (ER) and the host Golgi complex, with a distinctive membrane protein composition; involved in ER-to-Golgi transport. Sources: GOC:jl, GOC:pr Relationships: is a type of host intracellular membrane-bounded organelle [GO:0033648]; is a type of host cell cytoplasm part [GO:0033655] Also known as: host ER-Golgi intermediate compartment, host cell ER-Golgi intermediate compartment